low-density lipoprotein particle receptor binding [GO:0050750] (molecular function) Definition: Binding to a low-density lipoprotein receptor. Also known as: LDL receptor binding, low-density lipoprotein receptor binding Relationships: is a type of GO:0070325 Sources: GOC:ai